{
  "gene": "UniProtKB:Q6ZS02",
  "gene_symbol": "DNM1P46",
  "term_id": "UNKNOWN:0001",
  "term_label": "Unknown molecular function",
  "gene_name": "Putative GED domain-containing protein DNM1P46"
}